{
  "term_label": "G protein-coupled receptor activity",
  "gene_symbol": "ADGRG5",
  "term_id": "GO:0004930",
  "gene": "UniProtKB:Q8IZF4",
  "gene_name": "Adhesion G-protein coupled receptor G5"
}